positive regulation of immunoglobulin mediated immune response [GO:0002891] (biological process) Sources: GOC:add Definition: Any process that activates or increases the frequency, rate, or extent of an immunoglobulin mediated immune response. Subtypes: positive regulation of type III hypersensitivity [GO:0001805], positive regulation of type I hypersensitivity [GO:0001812], positive regulation of type II hypersensitivity [GO:0002894], GO:0002925, positive regulation of isotype switching [GO:0045830], positive regulation of immunoglobulin production in mucosal tissue [GO:2000558] Relationships: is a type of positive regulation of B cell mediated immunity [GO:0002714]; is a type of regulation of immunoglobulin mediated immune response [GO:0002889]; positively regulates immunoglobulin mediated immune response [GO:0016064] Also known as: up regulation of immunoglobulin mediated immune response, up-regulation of immunoglobulin mediated immune response, upregulation of immunoglobulin mediated immune response, activation of immunoglobulin mediated immune response, stimulation of immunoglobulin mediated immune response